{
  "term_label": "nucleus",
  "gene": "UniProtKB:Q9Y4B4",
  "gene_name": "Helicase ARIP4",
  "gene_symbol": "RAD54L2",
  "term_id": "GO:0005634"
}